{
  "gene_name": "Acid sphingomyelinase-like phosphodiesterase 3b",
  "term_label": "Unknown biological process",
  "gene": "UniProtKB:Q92485",
  "gene_symbol": "SMPDL3B",
  "term_id": "UNKNOWN:0002"
}